{
  "term_id": "GO:0010506",
  "term_label": "regulation of autophagy",
  "gene": "UniProtKB:O75385",
  "gene_symbol": "ULK1",
  "gene_name": "Serine_threonine-protein kinase ULK1"
}